{
  "gene_symbol": "FBXO46",
  "gene": "UniProtKB:Q6PJ61",
  "gene_name": "F-box only protein 46",
  "term_id": "UNKNOWN:0001",
  "term_label": "Unknown molecular function"
}